egasyn-beta-glucuronidase complex [GO:0070385] (CC) Relationships: is a type of endoplasmic reticulum protein-containing complex [GO:0140534] References: PMID:7744842 Definition: A protein complex that contains beta-glucuronidase and the carboxyl esterase egasyn; formation of the complex causes beta-glucuronidase to be retained in the endoplasmic reticulum.